glossopharyngeal nerve structural organization [GO:0021617] (biological process) Relationships: is a type of GO:0021604; is part of glossopharyngeal nerve morphogenesis [GO:0021615] Definition: The process that contributes to the act of creating the structural organization of the glossopharyngeal nerve. This process pertains to the physical shaping of a rudimentary structure. Various sensory and motor branches of the glossopharyngeal nerve supply nerve connections to the pharynx and back of the tongue. The branchial motor component contains motor fibers that innervate muscles that elevate the pharynx and larynx, and the tympanic branch supplies parasympathetic fibers to the otic ganglion. Sources: GOC:cls, GOC:dgh, GOC:dph, GOC:jid, GO_REF:0000021 Also known as: glossopharyngeal nerve structural organisation, CN IX structural organization